host apoplast [GO:0140593] (cellular component) Definition: The apoplast region surrounding a host plant cell. Plants may be described as having two major compartments: the living symplast and the non-living apoplast. The apoplast is external to the plasma membrane and includes cell walls, intercellular spaces and the lumen of dead structures such as xylem vessels. Water and solutes pass freely through it. The host is defined as the larger of the organisms involved in a symbiotic interaction. References: PMID:28082413 Also known as: host cell apoplast Relationships: is a type of host cell part [GO:0033643]